{
  "term_id": "GO:0048250",
  "gene_name": "Mitoferrin-1",
  "term_label": "iron import into the mitochondrion",
  "gene_symbol": "SLC25A37",
  "gene": "UniProtKB:Q9NYZ2"
}